{
  "term_id": "UNKNOWN:0003",
  "gene_name": "Protein CutA",
  "gene_symbol": "CUTA",
  "term_label": "Unknown cellular component",
  "gene": "UniProtKB:O60888"
}